{
  "gene_name": "Zinc finger protein 497",
  "gene": "UniProtKB:Q6ZNH5",
  "term_id": "UNKNOWN:0003",
  "gene_symbol": "ZNF497",
  "term_label": "Unknown cellular component"
}